{
  "gene_name": "E3 ubiquitin-protein ligase HECW1",
  "gene_symbol": "HECW1",
  "term_id": "GO:0005737",
  "term_label": "cytoplasm",
  "gene": "UniProtKB:Q76N89"
}